{
  "gene_symbol": "DEFB126",
  "term_id": "GO:0061844",
  "gene": "UniProtKB:Q9BYW3",
  "gene_name": "Beta-defensin 126",
  "term_label": "antimicrobial humoral immune response mediated by antimicrobial peptide"
}